response to pullulan [GO:0044592] (biological process) Regulation: regulated by regulation of response to pullulan [GO:1900518]; RO_0002212 by negative regulation of response to pullulan [GO:1900519]; positively regulated by positive regulation of response to pullulan [GO:1900520] Definition: A process that results in a change in state or activity of a cell (in terms of movement, secretion, enzyme production, gene expression, etc.) as a result of pullulan stimulus. Sources: GOC:mengo_curators, GOC:tt Relationships: is a type of response to carbohydrate [GO:0009743]